carpel development [GO:0048440] (biological process) Sources: GOC:go_curators Definition: The process whose specific outcome is the progression of the carpel over time, from its formation to the mature structure. A carpel is an organ (generally believed to be a modified foliar unit) at the centre of a flower, bearing one or more ovules and having its margins fused together or with other carpels to enclose the ovule in an ovary, and consisting also of a stigma and usually a style. Relationships: is a type of floral organ development [GO:0048437]; is_a phyllome development [GO:0048827]; is part of gynoecium development [GO:0048467]